{
  "term_label": "spindle",
  "term_id": "GO:0005819",
  "gene": "UniProtKB:P23258",
  "gene_name": "Tubulin gamma-1 chain",
  "gene_symbol": "TUBG1"
}